{
  "term_label": "plasma membrane",
  "term_id": "GO:0005886",
  "gene_name": "Vimentin",
  "gene_symbol": "VIM",
  "gene": "UniProtKB:P08670"
}